cell motility in response to calcium ion [GO:0097231] (biological process) Relationships: is a type of cell motility [GO:0048870]; is part of cellular response to calcium ion [GO:0071277] Also known as: Ca2+ facilitation of cell motility, calcium ion facilitation of cell motility References: PMID:19363786, PMID:21239624, PMID:8937985 Sources: GOC:pf Definition: Any process involved in the controlled self-propelled movement of a cell that results in translocation of the cell from one place to another as a result of a calcium ion stimulus.